{
  "gene": "UniProtKB:Q9NT22",
  "gene_symbol": "EMILIN3",
  "term_id": "UNKNOWN:0001",
  "term_label": "Unknown molecular function",
  "gene_name": "EMILIN-3"
}